{
  "gene_name": "Plexin-A3",
  "gene_symbol": "PLXNA3",
  "term_label": "regulation of cell migration",
  "term_id": "GO:0030334",
  "gene": "UniProtKB:P51805"
}